{
  "term_label": "proteolysis",
  "gene": "UniProtKB:Q9UKP5",
  "term_id": "GO:0006508",
  "gene_name": "A disintegrin and metalloproteinase with thrombospondin motifs 6",
  "gene_symbol": "ADAMTS6"
}